{
  "term_id": "GO:0042162",
  "gene_name": "CST complex subunit TEN1",
  "gene": "UniProtKB:Q86WV5",
  "term_label": "telomeric DNA binding",
  "gene_symbol": "TEN1"
}